{
  "gene_symbol": "RXRA",
  "term_label": "nervous system development",
  "term_id": "GO:0007399",
  "gene_name": "Retinoic acid receptor RXR-alpha",
  "gene": "UniProtKB:P19793"
}